flavonoid catabolic process [GO:0046275] (BP) Definition: The chemical reactions and pathways resulting in the breakdown of flavonoids, a group of phenolic derivatives containing a flavan skeleton. Sources: GOC:ai Also known as: flavonoid breakdown, flavonoid catabolism, flavonoid degradation Relationships: is a type of catabolic process [GO:0009056]; is a type of flavonoid metabolic process [GO:0009812] Subtypes: anthocyanin-containing compound catabolic process [GO:0046284], flavonoid phytoalexin catabolic process [GO:0046286], quercetin catabolic process [GO:1901733]